response to mercury ion [GO:0046689] (biological process) Relationships: is a type of response to metal ion [GO:0010038] Sources: GOC:ai Also known as: response to mercury, response to mercuric ion, mercuric sensitivity/resistance Definition: Any process that results in a change in state or activity of a cell or an organism (in terms of movement, secretion, enzyme production, gene expression, etc.) as a result of a mercury ion stimulus. Subtypes: cellular response to mercury ion [GO:0071288]